anaerobic cyclohexane-1-carboxylate catabolic process [GO:0010129] (biological process) Also known as: anaerobic cyclohexane-1-carboxylate breakdown, anaerobic cyclohexane-1-carboxylate catabolism, anaerobic cyclohexane-1-carboxylate degradation Sources: GOC:pz Definition: The chemical reactions and pathways resulting in the breakdown of cyclohexane-1-carboxylate, a alicyclic acid, in the absence of oxygen. Relationships: is a type of xenobiotic catabolic process [GO:0042178]